tyramine secretion, neurotransmission [GO:0061546] (biological process) Sources: GOC:dph Definition: The regulated release of a tyramine by a cell in which the tyramine acts as a neurotransmitter. Relationships: is a type of primary amine secretion, neurotransmission [GO:0061532]; is a type of GO:0061545